{
  "gene": "UniProtKB:Q6IMN6",
  "term_id": "GO:0005102",
  "term_label": "signaling receptor binding",
  "gene_symbol": "CAPRIN2",
  "gene_name": "Caprin-2"
}